auxin import into cell [GO:0060919] (biological process) Relationships: is a type of auxin transport [GO:0060918]; is a type of GO:0098739 Also known as: auxin influx References: PMID:22773749 Definition: The directed movement of auxins from outside of a cell into a cell.